{
  "gene": "UniProtKB:P0DJD9",
  "gene_symbol": "PGA5",
  "gene_name": "Pepsin A-5",
  "term_id": "UNKNOWN:0003",
  "term_label": "Unknown cellular component"
}